{
  "term_label": "RNA endonuclease activity",
  "gene": "UniProtKB:Q9UKV8",
  "gene_name": "Protein argonaute-2",
  "gene_symbol": "AGO2",
  "term_id": "GO:0004521"
}